{
  "gene_name": "Small ribosomal subunit protein uS15",
  "term_label": "Unknown biological process",
  "gene_symbol": "RPS13",
  "gene": "UniProtKB:P62277",
  "term_id": "UNKNOWN:0002"
}